{
  "gene_name": "LIM domain-binding protein 1",
  "term_label": "transcription coregulator activity",
  "gene_symbol": "LDB1",
  "gene": "UniProtKB:Q86U70",
  "term_id": "GO:0003712"
}